{
  "term_label": "Unknown molecular function",
  "term_id": "UNKNOWN:0001",
  "gene": "UniProtKB:Q9HBM1",
  "gene_name": "Kinetochore protein Spc25",
  "gene_symbol": "SPC25"
}